{
  "gene_name": "Tubulin polyglutamylase TTLL13",
  "term_id": "GO:0001578",
  "gene_symbol": "TTLL13",
  "term_label": "microtubule bundle formation",
  "gene": "UniProtKB:A6NNM8"
}